ERK5 cascade [GO:0070375] (biological process) Relationships: is a type of GO:0000165 Definition: A MAPK cascade containing at least the ERK5 MAP kinase (MAPK7; also called BMK1). It starts with the activation of a MAP3K, and the consecutive activation of a MPK2K and of ERK5. The cascade can also contain an additional tier: the upstream MAP4K. The kinases in each tier phosphorylate and activate the kinases in the downstream tier. The ERK5 cascade is activated by stress, mitogens, and by G protein-coupled receptors, and results in cellular responses such as cell growth, cell differentiation and development. Regulation: regulated by regulation of ERK5 cascade [GO:0070376]; negatively regulated by negative regulation of ERK5 cascade [GO:0070377]; positively regulated by positive regulation of ERK5 cascade [GO:0070378] References: PMID:16376520, PMID:16880823, PMID:20811974, PMID:23125017, PMID:28903453 Also known as: BMK cascade, BMK signaling pathway, BMK signalling pathway, BMK1 cascade, ERK5 signaling pathway, MAPK7 cascade, big MAP kinase signaling cascade, extracellular signal-regulated kinase 5 cascade